{
  "gene_symbol": "CDA",
  "term_label": "Unknown biological process",
  "term_id": "UNKNOWN:0002",
  "gene_name": "Cytidine deaminase",
  "gene": "UniProtKB:P32320"
}